{
  "gene_symbol": "RPS4Y1",
  "term_id": "GO:0003735",
  "gene_name": "Small ribosomal subunit protein eS4, Y isoform 1",
  "gene": "UniProtKB:P22090",
  "term_label": "structural constituent of ribosome"
}